{
  "gene_name": "Histone H2B type 2-K1",
  "gene_symbol": "H2BK1",
  "term_label": "nucleus",
  "term_id": "GO:0005634",
  "gene": "UniProtKB:A0A2R8Y619"
}